pollen adhesion [GO:0009876] (biological process) Definition: The process in which pollen deposited on the stigma adheres to cells of the stigma. Relationships: is a type of cell-cell adhesion [GO:0098609]; is part of pollen-pistil interaction [GO:0009875] Sources: GOC:tair_curators